{
  "gene_symbol": "RPH3A",
  "gene": "UniProtKB:Q9Y2J0",
  "term_id": "GO:0099502",
  "term_label": "calcium-dependent activation of synaptic vesicle fusion",
  "gene_name": "Rabphilin-3A"
}